ecdysone receptor signaling pathway [GO:0035076] (biological process) Sources: GOC:bf Relationships: is a type of GO:0030518; is part of cellular response to ecdysone [GO:0071390] Also known as: ecdysone receptor-mediated signalling pathway, nuclear receptor-mediated ecdysone signaling pathway Definition: A nuclear receptor-mediated signaling pathway initiated by an ecdysone binding to an intracellular receptor of the nuclear receptor protein family, and ending with regulation of a downstream cellular process, e.g. transcription. Regulation: regulated by regulation of ecdysone receptor signaling pathway [GO:0120141]; positively regulated by positive regulation of ecdysone receptor signaling pathway [GO:0120142]; negatively regulated by negative regulation of ecdysone receptor signaling pathway [GO:0120143]